lipoarabinomannan immune receptor activity [GO:0001877] (molecular function) Relationships: is a type of pattern recognition receptor activity [GO:0038187]; has part lipoarabinomannan binding [GO:0001876] Also known as: lipoarabinomannan receptor activity, LAM receptor activity Definition: Combining with lipoarabinomannan and transmitting the signal to initiate an innate immune response. References: PMID:10586073